{
  "gene": "UniProtKB:Q8WWV6",
  "gene_symbol": "FCAMR",
  "term_id": "GO:0005886",
  "term_label": "plasma membrane",
  "gene_name": "High affinity immunoglobulin alpha and immunoglobulin mu Fc receptor"
}